{
  "gene_name": "Olfactory receptor 4D11",
  "gene_symbol": "OR4D11",
  "term_label": "Unknown biological process",
  "term_id": "UNKNOWN:0002",
  "gene": "UniProtKB:Q8NGI4"
}